cyclic nucleotide metabolic process [GO:0009187] (biological process) Relationships: is a type of nucleotide metabolic process [GO:0009117] Subtypes: cyclic nucleotide biosynthetic process [GO:0009190], cyclic nucleotide catabolic process [GO:0009214], cyclic purine nucleotide metabolic process [GO:0052652] Also known as: cyclic nucleotide metabolism Definition: The chemical reactions and pathways involving a cyclic nucleotide, a nucleotide in which the phosphate group is in diester linkage to two positions on the sugar residue. Sources: GOC:go_curators, ISBN:0198506732